{
  "gene_symbol": "SEPTIN4",
  "gene_name": "Septin-4",
  "term_id": "GO:0032153",
  "gene": "UniProtKB:O43236",
  "term_label": "cell division site"
}